positive regulation of neuroinflammatory response [GO:0150078] (biological process) Sources: GOC:aruk, GOC:bc Relationships: is a type of GO:0050729; is a type of GO:0150077; positively regulates neuroinflammatory response [GO:0150076] Subtypes: positive regulation of astrocyte activation [GO:0061890], positive regulation of microglial cell activation [GO:1903980] Definition: Any process that activates or increases the frequency, rate or extent of neuroinflammatory response.